regulation of PSII associated light-harvesting complex II catabolic process [GO:0010550] (biological process) Relationships: is a type of regulation of protein catabolic process [GO:0042176]; regulates PSII associated light-harvesting complex II catabolic process [GO:0010304] Sources: GOC:dph, GOC:tb Also known as: regulation of LHCII catabolism, regulation of LHCII degradation Definition: Any process that modulates the chemical reactions and pathways resulting in the breakdown of one or more components of the light-harvesting complex of photosystem II.